{
  "gene_symbol": "GUCY1A2",
  "gene": "UniProtKB:P33402",
  "gene_name": "Guanylate cyclase soluble subunit alpha-2",
  "term_label": "guanylate cyclase complex, soluble",
  "term_id": "GO:0008074"
}